{
  "term_label": "serine-type endopeptidase inhibitor activity",
  "term_id": "GO:0004867",
  "gene_name": "Serine protease inhibitor Kazal-type 9",
  "gene_symbol": "SPINK9",
  "gene": "UniProtKB:Q5DT21"
}